{
  "gene": "UniProtKB:Q32ZL2",
  "gene_name": "Phospholipid phosphatase-related protein type 5",
  "term_label": "phosphatidate phosphatase activity",
  "term_id": "GO:0008195",
  "gene_symbol": "PLPPR5"
}